copper ion homeostasis [GO:0055070] (biological process) Subtypes: GO:0006878 Definition: Any process involved in the maintenance of an internal steady state of copper ions within an organism or cell. Relationships: is a type of GO:0055080; is a type of inorganic ion homeostasis [GO:0098771] Sources: GOC:ai, GOC:jid, GOC:mah Also known as: copper homeostasis